{
  "gene_name": "Ankyrin repeat domain-containing protein 65",
  "gene": "UniProtKB:E5RJM6",
  "gene_symbol": "ANKRD65",
  "term_id": "UNKNOWN:0003",
  "term_label": "Unknown cellular component"
}